protein localization to vacuole [GO:0072665] (biological process) Subtypes: protein targeting to vacuole [GO:0006623], protein transport to vacuole involved in ubiquitin-dependent protein catabolic process via the multivesicular body sorting pathway [GO:0043328], protein localization to lysosome [GO:0061462], protein localization to vacuolar membrane [GO:1903778] Relationships: is a type of GO:0033365 Definition: A process in which a protein is transported to, or maintained at, a location in a vacuole. Sources: GOC:ecd Also known as: protein localisation to vacuole